conidium formation [GO:0048315] (biological process) Regulation: regulated by regulation of conidium formation [GO:0075306]; positively regulated by positive regulation of conidium formation [GO:0075307]; negatively regulated by negative regulation of conidium formation [GO:0075308] Definition: The process of producing non-motile spores, called conidia, via mitotic asexual reproduction in higher fungi. Conidia are haploid cells genetically identical to their haploid parent. They are produced by conversion of hyphal elements, or are borne on sporogenous cells on or within specialized structures termed conidiophores, and participate in dispersal of the fungus. Relationships: is a type of asexual sporulation [GO:0030436]; is part of GO:0061794 Also known as: conidia formation, conidia biosynthesis Subtypes: arthrospore formation [GO:0034298], reproductive blastospore formation [GO:0034299] References: PMID:2524423, PMID:9529886 Sources: GOC:di, ISBN:0963117211